trans-synaptic signaling by BDNF [GO:0099191] (BP) Relationships: is a type of trans-synaptic signaling [GO:0099537] Also known as: trans-synaptic signaling by brain-derived neurotrophic factor Definition: Cell-cell signaling between presynapse and postsynapse mediated by brain-derived neurotrophic factor (BDNF) crossing the synaptic cleft. Subtypes: GO:0099183 Sources: GOC:dos